negative regulation of opsin-mediated signaling pathway [GO:0016059] (biological process) Subtypes: negative regulation of phospholipase C-activating phototransduction signaling pathway [GO:0016060] References: PMID:8316831 Definition: The process of restoring the photoreceptor cell to its unexcited state after termination of the stimulus (photon). Also known as: rod response recovery, deactivation of opsin mediated signaling, deactivation of rhodopsin mediated signalling, negative regulation of rhodopsin-mediated signaling pathway Relationships: is a type of regulation of opsin-mediated signaling pathway [GO:0022400]; is a type of negative regulation of response to external stimulus [GO:0032102]; is_a negative regulation of G protein-coupled receptor signaling pathway [GO:0045744]; negatively regulates G protein-coupled opsin signaling pathway [GO:0016056]